shikimate catabolic process [GO:0019633] (biological process) Relationships: is a type of shikimate metabolic process [GO:0019632]; is a type of GO:0072329 Definition: The chemical reactions and pathways resulting in the breakdown of shikimate, (3R,4S,5R)--3,4,5-trihydroxycyclohex-1-ene-1-carboxylate, the anion of shikimic acid. Also known as: shikimate breakdown, shikimate catabolism, shikimate degradation Sources: GOC:go_curators